{
  "gene": "UniProtKB:Q8TEA1",
  "term_label": "Unknown cellular component",
  "gene_symbol": "NSUN6",
  "gene_name": "tRNA (cytosine(72)-C(5))-methyltransferase NSUN6",
  "term_id": "UNKNOWN:0003"
}